{
  "gene_symbol": "PSMC3",
  "gene": "UniProtKB:P17980",
  "term_label": "proteasome-mediated ubiquitin-dependent protein catabolic process",
  "term_id": "GO:0043161",
  "gene_name": "26S proteasome regulatory subunit 6A"
}